{
  "term_id": "GO:0051607",
  "gene_symbol": "IFNL3",
  "gene": "UniProtKB:Q8IZI9",
  "gene_name": "Interferon lambda-3",
  "term_label": "defense response to virus"
}